rhamnetin 4'-O-methyltransferase activity [GO:0102448] (molecular function) Relationships: is a type of methyltransferase activity [GO:0008168] Definition: Catalysis of the reaction: rhamnetin + S-adenosyl-L-methionine = 7,4'-O-dimethylquercetin + H+ + S-adenosyl-L-homocysteine. Sources: RHEA:74731